ventral disc [GO:0097597] (cellular component) Definition: Specialized organelle found in Giardia species (trophozoite stage) and characterized by a spiral array of microtubules and microtubule-associated structures including dorsal microribbons and crossbridges. The edge of the ventral disc narrows into a lateral crest. The ventral disk mediates mechanical attachment of the trophozoite to the host's intestinal wall, and contains the contractile proteins actinin, alpha-actinin, myosin, and tropomyosin working towards contraction of the disk involved in adherence. References: PMID:11432808, PMID:4777416, PMID:5961344 Sources: GOC:giardia, ISBN:9780124260207 Relationships: is a type of GO:0043232; has part ventral disc lateral crest [GO:0097591]; has part ventral disc overlap zone [GO:0097592]; has part ventral disc dorsal microribbon [GO:0097594]; has part GO:0097595 Also known as: ventral adhesive disc, adhesive disc, ventral disk Note: Due to the asymmetric nature of the Giardia trophozoite, this term is defined spatially as the trophozoite is viewed from the dorsal side, with the two nuclei dorsal to the ventral disc, and the ventral disc toward the anterior.